{
  "gene_symbol": "FGF20",
  "gene_name": "Fibroblast growth factor 20",
  "gene": "UniProtKB:Q9NP95",
  "term_label": "cytoplasm",
  "term_id": "GO:0005737"
}